{
  "gene_symbol": "GLI4",
  "term_label": "Unknown cellular component",
  "gene_name": "Zinc finger protein GLI4",
  "term_id": "UNKNOWN:0003",
  "gene": "UniProtKB:P10075"
}